{
  "gene_name": "T-cell immunoreceptor with Ig and ITIM domains",
  "term_id": "GO:0032733",
  "gene_symbol": "TIGIT",
  "gene": "UniProtKB:Q495A1",
  "term_label": "positive regulation of interleukin-10 production"
}